heavy chain immunoglobulin complex [GO:0071762] (cellular component) Note: Note that a heavy chain immunoglobulin complex has the function of antigen binding if a suitable antigen is available. Note that IgNAR is found in serum of cartilaginous fish as a heavy chain dimer without immunoglobulin light chains. Note that HCab is found in camels as a heavy chain dimer without immunoglobulin light chains. Definition: A protein complex composed of two identical immunoglobulin heavy chains of the IgNAR isotype held together by disulfide bonds and lacking immunoglobulin light chains. Relationships: is a type of immunoglobulin complex [GO:0019814] References: PMID:12543123, PMID:16051357 Sources: GOC:add, ISBN:0781765196 Also known as: HCab, Ig NAR immunoglobulin complex, IgNAR antibody, IgNAR immunoglobulin complex